negative regulation of inositol phosphate biosynthetic process [GO:0010920] (biological process) Also known as: negative regulation of inositol phosphate biosynthesis Sources: GOC:dph, GOC:tb Definition: Any process that decreases the rate, frequency or extent of inositol phosphate biosynthesis. Inositol phosphate biosynthetic processes are the chemical reactions and pathways resulting in the formation of an inositol phosphate, 1,2,3,4,5,6-cyclohexanehexol, with one or more phosphate groups attached. Relationships: is a type of GO:0010919; is a type of negative regulation of carbohydrate metabolic process [GO:0045912]; is a type of negative regulation of phosphate metabolic process [GO:0045936]; is a type of negative regulation of alcohol biosynthetic process [GO:1902931]; RO_0002212 inositol phosphate biosynthetic process [GO:0032958] Subtypes: negative regulation of inositol trisphosphate biosynthetic process [GO:0032961]